{
  "term_label": "phospholipid binding",
  "term_id": "GO:0005543",
  "gene_name": "Pleckstrin homology domain-containing family A member 2",
  "gene": "UniProtKB:Q9HB19",
  "gene_symbol": "PLEKHA2"
}